{
  "term_label": "Unknown biological process",
  "gene_symbol": "SPRYD3",
  "term_id": "UNKNOWN:0002",
  "gene": "UniProtKB:Q8NCJ5",
  "gene_name": "SPRY domain-containing protein 3"
}